{
  "term_id": "GO:0005938",
  "gene_symbol": "ECT2",
  "term_label": "cell cortex",
  "gene_name": "Protein ECT2",
  "gene": "UniProtKB:Q9H8V3"
}